{
  "gene_name": "Uncharacterized protein",
  "term_label": "Unknown cellular component",
  "gene": "UniProtKB:A0A8V8TPP0",
  "gene_symbol": "A0A8V8TPP0",
  "term_id": "UNKNOWN:0003"
}